{
  "term_id": "GO:0000978",
  "gene": "UniProtKB:P0DKX0",
  "gene_symbol": "ZNF728",
  "term_label": "RNA polymerase II cis-regulatory region sequence-specific DNA binding",
  "gene_name": "Zinc finger protein 728"
}